{
  "gene_name": "Pumilio homolog 1",
  "gene_symbol": "PUM1",
  "term_label": "regulation of mRNA stability",
  "gene": "UniProtKB:Q14671",
  "term_id": "GO:0043488"
}